UDP-N-acetylgalactosamine-4-sulfate sulfotransferase activity [GO:0047368] (molecular function) Definition: Catalysis of the reaction: 3'-phospho-5'-adenylyl sulfate + UDP-N-acetyl-D-galactosamine 4-sulfate = adenosine 3',5'-diphosphate + H+ + UDP-N-acetyl-D-galactosamine 4,6-disulfate. Sources: EC:2.8.2.7, RHEA:14337 Also known as: UDP-N-acetylgalactosamine-4-sulphate sulphotransferase activity, 3'-phosphoadenylyl-sulfate:UDP-N-acetyl-D-galactosamine-4-sulfate 6-sulfotransferase activity, uridine diphospho-N-acetylgalactosamine 4-sulfate sulfotransferase activity, uridine diphosphoacetylgalactosamine 4-sulfate sulfotransferase activity Relationships: is a type of sulfotransferase activity [GO:0008146]